regulation of acute inflammatory response [GO:0002673] (biological process) Relationships: is a type of GO:0050727; regulates acute inflammatory response [GO:0002526] Definition: Any process that modulates the frequency, rate, or extent of an acute inflammatory response. Subtypes: regulation of kinin cascade [GO:0002256], Factor XII activation [GO:0002542], negative regulation of acute inflammatory response [GO:0002674], positive regulation of acute inflammatory response [GO:0002675], regulation of acute inflammatory response to antigenic stimulus [GO:0002864], negative regulation of B cell deletion [GO:0002868], positive regulation of B cell deletion [GO:0002869], negative regulation of natural killer cell tolerance induction [GO:0002872], GO:0002873, regulation of acute inflammatory response to non-antigenic stimulus [GO:0002877], regulation of fever generation [GO:0031620] Sources: GOC:add